{
  "term_id": "GO:0005783",
  "gene_symbol": "UGT1A4",
  "gene": "UniProtKB:P22310",
  "gene_name": "UDP-glucuronosyltransferase 1A4",
  "term_label": "endoplasmic reticulum"
}